basal tubulobulbar complex [GO:0061829] (CC) Definition: Actin-based structures involved in establishing the blood-testis barrier of the Sertoli cell. Relationships: is a type of GO:0036284 Also known as: basal TBC References: PMID:20403871, PMID:22510523